negative regulation of hormone secretion [GO:0046888] (biological process) Definition: Any process that stops, prevents, or reduces the frequency, rate or extent of the regulated release of a hormone from a cell. Also known as: down regulation of hormone secretion, down-regulation of hormone secretion, downregulation of hormone secretion, inhibition of hormone secretion Relationships: is a type of negative regulation of cell communication [GO:0010648]; is a type of GO:0023057; is a type of regulation of hormone secretion [GO:0046883]; is a type of negative regulation of secretion by cell [GO:1903531]; negatively regulates hormone secretion [GO:0046879] Subtypes: GO:0032277, negative regulation of activin secretion [GO:0032336], negative regulation of inhibin secretion [GO:0032339], negative regulation of juvenile hormone secretion [GO:0045972], negative regulation of adiponectin secretion [GO:0070164], negative regulation of peptide hormone secretion [GO:0090278], negative regulation of histamine secretion by mast cell [GO:1903594], GO:2000829, negative regulation of steroid hormone secretion [GO:2000832], negative regulation of androstenedione secretion [GO:2000838], negative regulation of dehydroepiandrosterone secretion [GO:2000841], negative regulation of testosterone secretion [GO:2000844] Sources: GOC:ai